{
  "gene": "UniProtKB:P51810",
  "term_id": "GO:0035643",
  "term_label": "L-DOPA receptor activity",
  "gene_name": "G-protein coupled receptor 143",
  "gene_symbol": "GPR143"
}